{
  "term_id": "GO:0014704",
  "gene_symbol": "CDH2",
  "term_label": "intercalated disc",
  "gene_name": "Cadherin-2",
  "gene": "UniProtKB:P19022"
}